{
  "term_id": "UNKNOWN:0003",
  "gene_symbol": "FAM87A",
  "gene_name": "Protein FAM87A",
  "term_label": "Unknown cellular component",
  "gene": "UniProtKB:P0C7U9"
}